{
  "gene": "UniProtKB:Q6UWP2",
  "gene_name": "Dehydrogenase_reductase SDR family member 11",
  "term_label": "Unknown cellular component",
  "term_id": "UNKNOWN:0003",
  "gene_symbol": "DHRS11"
}